L27 domain binding [GO:0097016] (molecular function) Definition: Binding to a L27 domain of a protein. L27 is composed of conserved negatively charged amino acids and a conserved aromatic amino acid. L27 domains can assemble proteins involved in signaling and establishment and maintenance of cell polarity into complexes by interacting in a heterodimeric manner. Relationships: is a type of protein domain specific binding [GO:0019904] References: PMID:15241471, PMID:17237226 Sources: GOC:BHF, Prosite:PDOC51022